regulation of metanephric S-shaped body morphogenesis [GO:2000004] (biological process) Relationships: is a type of regulation of animal organ morphogenesis [GO:2000027]; regulates metanephric S-shaped body morphogenesis [GO:0072284] Definition: Any process that modulates the frequency, rate or extent of metanephric S-shaped body morphogenesis. Subtypes: negative regulation of metanephric S-shaped body morphogenesis [GO:2000005] Sources: GOC:mtg_kidney_jan10, GOC:obol, GOC:yaf